{
  "term_label": "nucleus",
  "gene": "UniProtKB:Q8N988",
  "gene_symbol": "ZNF557",
  "term_id": "GO:0005634",
  "gene_name": "Zinc finger protein 557"
}